{
  "term_id": "UNKNOWN:0001",
  "gene": "UniProtKB:Q96AY4",
  "gene_name": "Tetratricopeptide repeat protein 28",
  "gene_symbol": "TTC28",
  "term_label": "Unknown molecular function"
}